{
  "gene": "UniProtKB:P00973",
  "gene_symbol": "OAS1",
  "gene_name": "2'-5'-oligoadenylate synthase 1",
  "term_id": "GO:0003725",
  "term_label": "double-stranded RNA binding"
}